angular vestibuloocular reflex [GO:0060006] (BP) Definition: A vestibular reflex by which a response to an angular acceleration stimulus begins with an afferent nerve impulse from a receptor in the semi-circular canal and ends with the compensatory action of eye muscles. Signaling never reaches a level of consciousness. References: PMID:11784757 Sources: GOC:dph Relationships: is a type of vestibular reflex [GO:0060005]